{
  "gene_symbol": "GNRHR2",
  "term_id": "GO:0032870",
  "gene_name": "Putative gonadotropin-releasing hormone II receptor",
  "term_label": "cellular response to hormone stimulus",
  "gene": "UniProtKB:Q96P88"
}